response to trichostatin A [GO:0035983] (BP) References: PMID:20181743 Sources: GOC:yaf Relationships: is a type of response to antibiotic [GO:0046677]; is a type of response to nitrogen compound [GO:1901698]; is a type of response to oxygen-containing compound [GO:1901700] Subtypes: cellular response to trichostatin A [GO:0035984] Definition: Any process that results in a change in state or activity of a cell or an organism (in terms of movement, secretion, enzyme production, gene expression, etc.) as a result of a trichostatin A stimulus.